{
  "term_id": "UNKNOWN:0001",
  "gene": "UniProtKB:Q6UE05",
  "gene_symbol": "TMEM270",
  "gene_name": "Transmembrane protein 270",
  "term_label": "Unknown molecular function"
}